{
  "gene_name": "Unconventional myosin-VI",
  "gene": "UniProtKB:Q9UM54",
  "term_label": "inner ear auditory receptor cell differentiation",
  "term_id": "GO:0042491",
  "gene_symbol": "MYO6"
}